{
  "term_label": "Unknown biological process",
  "gene_symbol": "MEX3D",
  "gene": "UniProtKB:Q86XN8",
  "term_id": "UNKNOWN:0002",
  "gene_name": "RNA-binding protein MEX3D"
}